{
  "term_id": "GO:0004961",
  "gene_symbol": "TBXA2R",
  "term_label": "thromboxane A2 receptor activity",
  "gene_name": "Thromboxane A2 receptor",
  "gene": "UniProtKB:P21731"
}